{
  "gene_name": "G2 and S phase-expressed protein 1",
  "term_id": "GO:0005881",
  "gene_symbol": "GTSE1",
  "term_label": "cytoplasmic microtubule",
  "gene": "UniProtKB:Q9NYZ3"
}